helvolic acid catabolic process [GO:1900811] (biological process) Relationships: is a type of GO:0006706; is a type of ketone catabolic process [GO:0042182]; is a type of carboxylic acid catabolic process [GO:0046395]; is a type of secondary metabolite catabolic process [GO:0090487]; is a type of GO:0120256 Sources: GOC:TermGenie, GOC:di Also known as: helvolic acid breakdown, helvolic acid catabolism, helvolic acid degradation, Fumigacin breakdown, Fumigacin catabolic process, Fumigacin catabolism, Fumigacin degradation Definition: The chemical reactions and pathways resulting in the breakdown of helvolic acid.